{
  "gene": "UniProtKB:Q9Y426",
  "term_id": "UNKNOWN:0002",
  "gene_name": "C2 domain-containing protein 2",
  "term_label": "Unknown biological process",
  "gene_symbol": "C2CD2"
}